{
  "gene": "UniProtKB:P17706",
  "term_id": "GO:0004726",
  "term_label": "non-membrane spanning protein tyrosine phosphatase activity",
  "gene_name": "Tyrosine-protein phosphatase non-receptor type 2",
  "gene_symbol": "PTPN2"
}